magnetosome lumen [GO:0110145] (cellular component) Relationships: is a type of GO:0070013; is part of GO:0110143 Definition: The volume enclosed by the membrane of a magnetosome. References: PMID:27620945 Sources: GOC:aa